{
  "gene_symbol": "SNCA",
  "gene_name": "Alpha-synuclein",
  "term_id": "GO:0030672",
  "gene": "UniProtKB:P37840",
  "term_label": "synaptic vesicle membrane"
}